{
  "gene_symbol": "PYCARD",
  "gene_name": "Apoptosis-associated speck-like protein containing a CARD",
  "term_id": "GO:0097193",
  "term_label": "intrinsic apoptotic signaling pathway",
  "gene": "UniProtKB:Q9ULZ3"
}